{
  "gene_symbol": "SLC7A1",
  "term_label": "L-arginine transmembrane transporter activity",
  "gene_name": "High affinity cationic amino acid transporter 1",
  "term_id": "GO:0061459",
  "gene": "UniProtKB:P30825"
}